sterol catabolic process [GO:0016127] (biological process) Subtypes: cholesterol catabolic process [GO:0006707], ecdysone catabolic process [GO:0006708] Relationships: is a type of steroid catabolic process [GO:0006706]; is a type of sterol metabolic process [GO:0016125] Also known as: sterol breakdown, sterol catabolism, sterol degradation Definition: The chemical reactions and pathways resulting in the breakdown of sterols, steroids with one or more hydroxyl groups and a hydrocarbon side-chain in the molecule. Sources: GOC:go_curators